{
  "gene_symbol": "BPIFB1",
  "term_id": "GO:0034144",
  "gene": "UniProtKB:Q8TDL5",
  "term_label": "negative regulation of toll-like receptor 4 signaling pathway",
  "gene_name": "BPI fold-containing family B member 1"
}